{
  "term_label": "protein-membrane adaptor activity",
  "term_id": "GO:0043495",
  "gene_symbol": "VAPB",
  "gene_name": "Vesicle-associated membrane protein-associated protein B_C",
  "gene": "UniProtKB:O95292"
}